{
  "term_label": "oxygen transport",
  "term_id": "GO:0015671",
  "gene": "UniProtKB:P02008",
  "gene_name": "Hemoglobin subunit zeta",
  "gene_symbol": "HBZ"
}